{
  "gene_symbol": "TMPRSS9",
  "gene": "UniProtKB:Q7Z410",
  "term_id": "GO:0031639",
  "term_label": "plasminogen activation",
  "gene_name": "Transmembrane protease serine 9"
}